cytoplasmic replisome [GO:0043600] (cellular component) Relationships: is a type of replisome [GO:0030894]; BFO_0000050 cytoplasmic replication fork [GO:0043597]; has part DNA polymerase III complex [GO:0009360]; has part single-stranded DNA-binding protein complex [GO:0044777] Sources: GOC:jl, GOC:mtg_sensu Definition: A multi-component enzymatic machine at the cytoplasmic replication fork, which mediates DNA replication. Includes DNA primase, DNA polymerase, DNA helicase, and other proteins. Also known as: prokaryotic replisome